{
  "term_id": "GO:0032911",
  "term_label": "negative regulation of transforming growth factor beta1 production",
  "gene": "UniProtKB:O43914",
  "gene_name": "TYRO protein tyrosine kinase-binding protein",
  "gene_symbol": "TYROBP"
}